{
  "gene": "UniProtKB:Q6NYC1",
  "term_label": "P-TEFb complex binding",
  "gene_name": "Bifunctional arginine demethylase and lysyl-hydroxylase JMJD6",
  "term_id": "GO:0106140",
  "gene_symbol": "JMJD6"
}